{
  "term_id": "GO:0006829",
  "term_label": "zinc ion transport",
  "gene_symbol": "SLC30A6",
  "gene": "UniProtKB:Q6NXT4",
  "gene_name": "Zinc transporter 6"
}